{
  "term_label": "nucleus",
  "gene_symbol": "MAGEA12",
  "term_id": "GO:0005634",
  "gene": "UniProtKB:P43365",
  "gene_name": "Melanoma-associated antigen 12"
}